{
  "gene": "UniProtKB:Q13191",
  "gene_name": "E3 ubiquitin-protein ligase CBL-B",
  "term_label": "receptor tyrosine kinase binding",
  "term_id": "GO:0030971",
  "gene_symbol": "CBLB"
}